positive regulation of viral life cycle [GO:1903902] (biological process) Relationships: is a type of positive regulation of viral process [GO:0048524]; is a type of regulation of viral life cycle [GO:1903900]; positively regulates GO:0019058 References: PMID:18005716 Sources: GOC:TermGenie, GO_REF:0000058 Subtypes: positive regulation of viral entry into host cell [GO:0046598], positive regulation of intracellular transport of viral material [GO:1901254], positive regulation of receptor-mediated virion attachment to host cell [GO:1902736], positive regulation of viral budding via host ESCRT complex [GO:1903774], GO:1905138 Definition: Any process that activates or increases the frequency, rate or extent of viral life cycle. Also known as: up regulation of viral life cycle, up-regulation of viral life cycle, upregulation of viral life cycle, activation of viral assembly, maturation, egress, and release, activation of viral life cycle, positive regulation of viral assembly, maturation, egress, and release, up regulation of viral assembly, maturation, egress, and release, up-regulation of viral assembly, maturation, egress, and release, upregulation of viral assembly, maturation, egress, and release, activation of lytic viral life cycle, activation of viral infectious cycle, activation of viral replication, positive regulation of lytic viral life cycle, positive regulation of viral infectious cycle, positive regulation of viral replication, up regulation of lytic viral life cycle, up regulation of viral infectious cycle, up regulation of viral replication, up-regulation of lytic viral life cycle, up-regulation of viral infectious cycle, up-regulation of viral replication, upregulation of lytic viral life cycle, upregulation of viral infectious cycle, upregulation of viral replication